{
  "gene_symbol": "AFG2B",
  "term_id": "GO:0030970",
  "gene_name": "ATPase family gene 2 protein homolog B",
  "term_label": "retrograde protein transport, ER to cytosol",
  "gene": "UniProtKB:Q9BVQ7"
}